{
  "term_id": "GO:0046036",
  "gene": "UniProtKB:Q9Y227",
  "term_label": "CTP metabolic process",
  "gene_symbol": "ENTPD4",
  "gene_name": "Ectonucleoside triphosphate diphosphohydrolase 4"
}